{
  "gene_name": "Medium-chain specific acyl-CoA dehydrogenase, mitochondrial",
  "term_label": "medium-chain fatty acid catabolic process",
  "gene": "UniProtKB:P11310",
  "term_id": "GO:0051793",
  "gene_symbol": "ACADM"
}